{
  "gene": "UniProtKB:Q8WUA8",
  "gene_symbol": "TSKU",
  "term_id": "UNKNOWN:0002",
  "gene_name": "Tsukushi",
  "term_label": "Unknown biological process"
}